{
  "gene_symbol": "UNC13B",
  "gene_name": "Protein unc-13 homolog B",
  "gene": "UniProtKB:O14795",
  "term_id": "GO:0042734",
  "term_label": "presynaptic membrane"
}